{
  "gene_symbol": "RAET1G",
  "term_label": "positive regulation of T cell mediated cytotoxicity",
  "term_id": "GO:0001916",
  "gene": "UniProtKB:Q6H3X3",
  "gene_name": "UL-16 binding protein 5"
}